{
  "term_label": "Unknown cellular component",
  "gene": "UniProtKB:Q5W064",
  "gene_name": "Lipase member J",
  "gene_symbol": "LIPJ",
  "term_id": "UNKNOWN:0003"
}